{
  "term_label": "regulation of transcription by RNA polymerase II",
  "gene": "UniProtKB:Q01196",
  "gene_name": "Runt-related transcription factor 1",
  "term_id": "GO:0006357",
  "gene_symbol": "RUNX1"
}